{
  "gene_symbol": "CD99L2",
  "term_label": "Unknown molecular function",
  "gene": "UniProtKB:Q8TCZ2",
  "term_id": "UNKNOWN:0001",
  "gene_name": "CD99 antigen-like protein 2"
}